asymmetric, glutamatergic, excitatory synapse [GO:0098985] (CC) Definition: A neuron to neuron synapse with a postsynaptic density, that uses glutamate as a neurotransmitter and whose activity results in excitatory postsynaptic potentials. Subtypes: cerebellar granule cell to Purkinje cell synapse [GO:0150048], GO:0150053 Sources: GOC:dos Relationships: is a type of asymmetric synapse [GO:0032279]; is a type of excitatory synapse [GO:0060076]; is_a glutamatergic synapse [GO:0098978]